{
  "gene_symbol": "TMPRSS7",
  "gene_name": "Transmembrane protease serine 7",
  "term_label": "protein processing",
  "term_id": "GO:0016485",
  "gene": "UniProtKB:Q7RTY8"
}